{
  "gene_name": "Ras-related protein Rab-39A",
  "term_label": "phagosome-lysosome fusion",
  "gene": "UniProtKB:Q14964",
  "term_id": "GO:0090385",
  "gene_symbol": "RAB39A"
}